{
  "gene_symbol": "PPP4R3C",
  "gene": "UniProtKB:Q6ZMV5",
  "gene_name": "Protein PPP4R3C",
  "term_id": "GO:0006974",
  "term_label": "DNA damage response"
}